{
  "term_id": "GO:0005615",
  "gene_name": "Peptidase inhibitor 15",
  "gene": "UniProtKB:O43692",
  "gene_symbol": "PI15",
  "term_label": "extracellular space"
}